{
  "term_label": "Unknown molecular function",
  "gene_symbol": "C1QL2",
  "term_id": "UNKNOWN:0001",
  "gene": "UniProtKB:Q7Z5L3",
  "gene_name": "Complement C1q-like protein 2"
}